{
  "gene": "UniProtKB:Q3KP66",
  "term_label": "Unknown molecular function",
  "term_id": "UNKNOWN:0001",
  "gene_name": "Innate immunity activator protein",
  "gene_symbol": "INAVA"
}